benzoyl-CoA reductase activity [GO:0018522] (molecular function) Also known as: cyclohexa-1,5-diene-1-carbonyl-CoA:ferredoxin oxidoreductase (aromatizing, ATP-forming) activity, benzoyl-CoA reductase (dearomatizing) activity Sources: EC:1.3.7.8 Relationships: is a type of oxidoreductase activity, acting on the CH-CH group of donors, iron-sulfur protein as acceptor [GO:0016636] Definition: Catalysis of the reaction: 2 ADP + cyclohexa-1,5-diene-1-carbonyl-CoA + oxidized ferredoxin + 2 phosphate = 2 ATP + 2 H2O + benzoyl-CoA + reduced ferredoxin.